{
  "term_label": "synaptic vesicle membrane",
  "gene": "UniProtKB:O43761",
  "gene_name": "Synaptogyrin-3",
  "term_id": "GO:0030672",
  "gene_symbol": "SYNGR3"
}